{
  "term_id": "GO:0005886",
  "gene": "UniProtKB:Q86YM7",
  "term_label": "plasma membrane",
  "gene_name": "Homer protein homolog 1",
  "gene_symbol": "HOMER1"
}